{
  "gene": "UniProtKB:Q86XE3",
  "term_label": "calcium import into the mitochondrion",
  "term_id": "GO:0036444",
  "gene_symbol": "MICU3",
  "gene_name": "Calcium uptake protein 3, mitochondrial"
}